{
  "term_label": "Unknown biological process",
  "gene_symbol": "KRTAP26-1",
  "term_id": "UNKNOWN:0002",
  "gene_name": "Keratin-associated protein 26-1",
  "gene": "UniProtKB:Q6PEX3"
}